receptor-mediated endocytosis involved in cholesterol transport [GO:0090118] (biological process) Definition: A receptor-mediated endocytosis process involved in intracellular cholesterol transport. Sources: GOC:ascb_2009, GOC:dph, GOC:pr, GOC:tb Also known as: receptor-mediated endocytosis involved in intracellular cholesterol transport, receptor-mediated endocytosis of LDL, receptor-mediated endocytosis of low-density lipoprotein involved in cholesterol transport, receptor-mediated endocytosis of low-density lipoprotein particle involved in cholesterol transport Regulation: regulated by regulation of receptor-mediated endocytosis involved in cholesterol transport [GO:1905600]; negatively regulated by GO:1905601; RO_0002213 by positive regulation of receptor-mediated endocytosis involved in cholesterol transport [GO:1905602] Relationships: is a type of receptor-mediated endocytosis [GO:0006898]; is a type of intracellular transport [GO:0046907]; is part of intracellular cholesterol transport [GO:0032367]